{
  "gene_name": "Clarin-3",
  "gene": "UniProtKB:Q8NCR9",
  "term_id": "UNKNOWN:0003",
  "gene_symbol": "CLRN3",
  "term_label": "Unknown cellular component"
}